monoamine transport [GO:0015844] (biological process) Sources: GOC:mah Definition: The directed movement of monoamines, organic compounds that contain one amino group that is connected to an aromatic ring by an ethylene group (-CH2-CH2-), into, out of or within a cell, or between cells, by means of some agent such as a transporter or pore. Subtypes: serotonin transport [GO:0006837], catecholamine transport [GO:0051937], GO:0061545 Relationships: is a type of nitrogen compound transport [GO:0071705]